{
  "gene_symbol": "RACGAP1",
  "term_id": "GO:0000281",
  "term_label": "mitotic cytokinesis",
  "gene_name": "Rac GTPase-activating protein 1",
  "gene": "UniProtKB:Q9H0H5"
}